{
  "gene": "UniProtKB:Q9UN79",
  "term_id": "GO:0000981",
  "gene_symbol": "SOX13",
  "term_label": "DNA-binding transcription factor activity, RNA polymerase II-specific",
  "gene_name": "Transcription factor SOX-13"
}